protein hexamerization [GO:0034214] (biological process) Sources: GOC:ecd Relationships: is_a protein complex oligomerization [GO:0051259] Definition: The formation of a protein hexamer, a macromolecular structure consisting of six noncovalently associated identical or nonidentical subunits. Also known as: protein hexamer assembly, protein hexamer biosynthesis, protein hexamer biosynthetic process, protein hexamer formation